negative regulation of snoRNA metabolic process [GO:1903324] (biological process) Sources: GOC:TermGenie, GOC:vw, GO_REF:0000058 Relationships: is a type of negative regulation of RNA metabolic process [GO:0051253]; is a type of regulation of snoRNA metabolic process [GO:1903323]; negatively regulates sno(s)RNA metabolic process [GO:0016074] Definition: Any process that stops, prevents or reduces the frequency, rate or extent of snoRNA metabolic process. Also known as: down regulation of snoRNA metabolic process, down regulation of snoRNA metabolism, down-regulation of snoRNA metabolic process, down-regulation of snoRNA metabolism, downregulation of snoRNA metabolic process, downregulation of snoRNA metabolism, negative regulation of snoRNA metabolism, inhibition of snoRNA metabolic process, inhibition of snoRNA metabolism Subtypes: negative regulation of snoRNA processing [GO:1902797]